regulation of pseudohyphal septin ring assembly [GO:0062164] (biological process) Subtypes: positive regulation of pseudohyphal septin ring assembly [GO:0062165], negative regulation of pseudohyphal septin ring assembly [GO:0062166] Definition: Any process that modulates the rate, frequency or extent of pseudohyphal septin ring assembly. Relationships: is a type of regulation of protein-containing complex assembly [GO:0043254]; is a type of regulation of cytoskeleton organization [GO:0051493]; is a type of regulation of organelle assembly [GO:1902115]; RO_0002211 GO:0062163 References: PMID:29567712